regulation of intrinsic apoptotic signaling pathway [GO:2001242] (biological process) Sources: GOC:mtg_apoptosis Subtypes: regulation of oxidative stress-induced intrinsic apoptotic signaling pathway [GO:1902175], regulation of intrinsic apoptotic signaling pathway in response to osmotic stress [GO:1902218], regulation of intrinsic apoptotic signaling pathway in response to DNA damage [GO:1902229], regulation of endoplasmic reticulum stress-induced intrinsic apoptotic signaling pathway [GO:1902235], GO:1902253, regulation of hypoxia-induced intrinsic apoptotic signaling pathway [GO:1903297], GO:1905258, negative regulation of intrinsic apoptotic signaling pathway [GO:2001243], GO:2001244 Also known as: regulation of intrinsic apoptotic pathway, regulation of intrinsic apoptotic signalling pathway, regulation of mitochondrial-mediated apoptotic pathway, regulation of intrinsic apoptosis Definition: Any process that modulates the frequency, rate or extent of intrinsic apoptotic signaling pathway. Relationships: is a type of GO:1902531; is a type of regulation of apoptotic signaling pathway [GO:2001233]; regulates intrinsic apoptotic signaling pathway [GO:0097193]